regulation of axon extension [GO:0030516] (biological process) Definition: Any process that modulates the rate, direction or extent of axon extension. Subtypes: negative regulation of axon extension [GO:0030517], positive regulation of axon extension [GO:0045773], GO:0048690, regulation of axon extension involved in axon guidance [GO:0048841] Relationships: is a type of regulation of developmental growth [GO:0048638]; is a type of regulation of extent of cell growth [GO:0061387]; regulates axon extension [GO:0048675] Sources: GOC:go_curators